{
  "gene_name": "Brain and acute leukemia cytoplasmic protein",
  "gene": "UniProtKB:Q8WXS3",
  "term_label": "cytoplasm",
  "term_id": "GO:0005737",
  "gene_symbol": "BAALC"
}